{
  "term_id": "GO:0005886",
  "term_label": "plasma membrane",
  "gene": "UniProtKB:P14416",
  "gene_name": "D(2) dopamine receptor",
  "gene_symbol": "DRD2"
}